response to ethylene [GO:0009723] (biological process) Relationships: is a type of response to hormone [GO:0009725] Subtypes: detection of ethylene stimulus [GO:0009727], cellular response to ethylene stimulus [GO:0071369] Sources: GOC:jl Also known as: response to ethene stimulus, response to ethylene stimulus Definition: Any process that results in a change in state or activity of a cell or an organism (in terms of movement, secretion, enzyme production, gene expression, etc.) as a result of an ethylene (ethene) stimulus.